(25S)-Delta(7)-dafachronate metabolic process [GO:1902056] (biological process) References: PMID:22505847 Sources: GOC:TermGenie Definition: The chemical reactions and pathways involving (25S)-Delta(7)-dafachronate. Also known as: (25S)-Delta(7)-dafachronate metabolism Relationships: is a type of steroid metabolic process [GO:0008202]; is a type of carboxylic acid metabolic process [GO:0019752]; is a type of ketone metabolic process [GO:0042180]